assembly of actomyosin apparatus involved in mitotic cytokinesis [GO:1902407] (biological process) Sources: GOC:TermGenie, GOC:mtg_cell_cycle Also known as: actomyosin apparatus assembly involved in cytokinesis involved in mitotic cell cycle, cytokinesis, formation of actomyosin apparatus involved in mitotic cell cycle, formation of actomyosin apparatus involved in cytokinesis involved in mitotic cell cycle Subtypes: phragmoplast assembly [GO:0000914], mitotic actomyosin contractile ring assembly [GO:1903475] Relationships: is a type of assembly of actomyosin apparatus involved in cytokinesis [GO:0000912]; is a type of mitotic cytokinetic process [GO:1902410] Definition: Any assembly of mitotic cytokinetic actomyosin apparatus.